spliceosomal complex disassembly [GO:0000390] (BP) Definition: Disassembly of a spliceosomal complex with the ATP-dependent release of the product RNAs, one of which is composed of the joined exons. In cis splicing, the other product is the excised sequence, often a single intron, in a lariat structure. Also known as: spliceosome disassembly, spliceosome complex disassembly, U12-type spliceosome disassembly, U2-type spliceosome disassembly Sources: GOC:krc, ISBN:0879695897 Relationships: is a type of protein-RNA complex disassembly [GO:0032988]; is part of GO:0000398